{
  "gene_symbol": "UBE2D3",
  "gene_name": "Ubiquitin-conjugating enzyme E2 D3",
  "term_label": "ubiquitin-dependent protein catabolic process",
  "term_id": "GO:0006511",
  "gene": "UniProtKB:P61077"
}